{
  "gene": "UniProtKB:Q86SP6",
  "gene_symbol": "GPR149",
  "term_label": "G protein-coupled receptor activity",
  "term_id": "GO:0004930",
  "gene_name": "Probable G-protein coupled receptor 149"
}